carnitine 3-dehydrogenase activity [GO:0047728] (molecular function) Definition: Catalysis of the reaction: carnitine + NAD+ = 3-dehydrocarnitine + H+ + NADH. Sources: EC:1.1.1.108, RHEA:19265 Also known as: carnitine:NAD+ 3-oxidoreductase activity Relationships: is a type of oxidoreductase activity, acting on the CH-OH group of donors, NAD or NADP as acceptor [GO:0016616]